guanine transport [GO:0015854] (biological process) Relationships: is a type of purine nucleobase transport [GO:0006863] Sources: GOC:go_curators Subtypes: guanine transmembrane transport [GO:1903716] Definition: The directed movement of guanine, 2-amino-6-hydroxypurine, into, out of or within a cell, or between cells, by means of some agent such as a transporter or pore.